negative regulation of sodium ion transport [GO:0010766] (biological process) Relationships: is a type of regulation of sodium ion transport [GO:0002028]; is a type of negative regulation of monoatomic ion transport [GO:0043271]; RO_0002212 sodium ion transport [GO:0006814] Sources: GOC:dph, GOC:tb Definition: Any process that decreases the frequency, rate or extent of the directed movement of sodium ions (Na+) into, out of or within a cell, or between cells, by means of some agent such as a transporter or pore. Subtypes: negative regulation of sodium ion transmembrane transport [GO:1902306]